{
  "term_label": "structural constituent of tooth enamel",
  "gene": "UniProtKB:Q9NRM1",
  "term_id": "GO:0030345",
  "gene_symbol": "ENAM",
  "gene_name": "Enamelin"
}